S-methylmethionine biosynthetic process [GO:0010250] (biological process) Definition: The chemical reactions and pathways resulting in the formation of S-methyl-methionine (SMM) from methionine and S-adenosyl-methionine (Ado-Met), catalyzed by methionine S-methyltransferase (MMT). SMM can be reconverted to methionine by donating a methyl group to homocysteine, and concurrent operation of this reaction and that mediated by MMT sets up the SMM cycle. References: PMID:12692340 Also known as: S-methylmethionine anabolism, S-methylmethionine biosynthesis, S-methylmethionine formation, S-methylmethionine synthesis Relationships: is a type of S-methylmethionine metabolic process [GO:0033477]; is a type of modified amino acid biosynthetic process [GO:0042398]; is a type of GO:0044272